podosome ring [GO:0061826] (cellular component) Definition: The ring structure surrounding the podosome core, containing proteins such as vinculin and talin. Relationships: is a type of cellular anatomical structure [GO:0110165]; is part of podosome [GO:0002102] References: PMID:23158496